{
  "term_label": "mRNA binding",
  "gene_name": "mRNA-decapping enzyme 1A",
  "term_id": "GO:0003729",
  "gene_symbol": "DCP1A",
  "gene": "UniProtKB:Q9NPI6"
}